{
  "term_id": "UNKNOWN:0002",
  "gene_symbol": "LINC01549",
  "gene": "UniProtKB:A6NIU2",
  "gene_name": "Putative uncharacterized protein encoded by LINC01549",
  "term_label": "Unknown biological process"
}